{
  "term_id": "UNKNOWN:0003",
  "term_label": "Unknown cellular component",
  "gene_symbol": "CCDC43",
  "gene": "UniProtKB:Q96MW1",
  "gene_name": "Coiled-coil domain-containing protein 43"
}